{
  "term_label": "extracellular matrix",
  "gene": "UniProtKB:P39060",
  "term_id": "GO:0031012",
  "gene_symbol": "COL18A1",
  "gene_name": "Collagen alpha-1(XVIII) chain"
}